detection of external stimulus [GO:0009581] (biological process) Sources: GOC:hb Definition: The series of events in which an external stimulus is received by a cell and converted into a molecular signal. Subtypes: detection of light stimulus [GO:0009583], detection of gravity [GO:0009590], detection of wounding [GO:0014822], detection of temperature stimulus [GO:0016048], detection of mechanical stimulus [GO:0050982], detection of humidity [GO:0098513] Also known as: perception of external stimulus Relationships: is a type of response to external stimulus [GO:0009605]; is a type of detection of stimulus [GO:0051606]